interleukin-2 binding [GO:0019976] (molecular function) Definition: Binding to interleukin-2. Relationships: is a type of GO:0019838; is_a cytokine binding [GO:0019955] Sources: GOC:jl Also known as: IL-2 binding